CHRAC [GO:0008623] (cellular component) Definition: An ISWI complex that contains an ATPase subunit of the ISWI family (SNF2H in mammals, Isw2 in S. cerevisiae), an ACF1 homolog, and additional small histone fold subunits (generally two of these, but Xenopus has only one and some additional non-conserved subunits). CHRAC plays roles in the regulation of RNA polymerase II transcription and in DNA replication and repair. Relationships: is a type of GO:0031010 References: PMID:15284901, PMID:16568949, PMID:21810179, PMID:9252192 Sources: GOC:bf, GOC:krc Also known as: chromatin accessibility complex, ISW2 complex